{
  "term_id": "GO:0000981",
  "gene": "UniProtKB:P52945",
  "term_label": "DNA-binding transcription factor activity, RNA polymerase II-specific",
  "gene_name": "Pancreas_duodenum homeobox protein 1",
  "gene_symbol": "PDX1"
}